{
  "gene": "UniProtKB:P0DI80",
  "gene_symbol": "SMIM6",
  "gene_name": "Small integral membrane protein 6",
  "term_id": "UNKNOWN:0002",
  "term_label": "Unknown biological process"
}